{
  "gene": "UniProtKB:Q5HY98",
  "term_label": "DNA-binding transcription factor activity, RNA polymerase II-specific",
  "gene_symbol": "ZNF766",
  "term_id": "GO:0000981",
  "gene_name": "Zinc finger protein 766"
}